{
  "gene_symbol": "ELAVL3",
  "gene": "UniProtKB:Q14576",
  "term_label": "Unknown cellular component",
  "gene_name": "ELAV-like protein 3",
  "term_id": "UNKNOWN:0003"
}